{
  "term_id": "GO:0005737",
  "gene_name": "Ribosomal protein S6 kinase alpha-4",
  "gene_symbol": "RPS6KA4",
  "gene": "UniProtKB:O75676",
  "term_label": "cytoplasm"
}